{
  "gene_name": "Tripartite motif-containing protein 66",
  "gene_symbol": "TRIM66",
  "term_id": "GO:0000785",
  "gene": "UniProtKB:O15016",
  "term_label": "chromatin"
}